{
  "gene_symbol": "ZNF320",
  "term_label": "nucleus",
  "gene": "UniProtKB:A2RRD8",
  "term_id": "GO:0005634",
  "gene_name": "Zinc finger protein 320"
}